mycolic acid biosynthetic process [GO:0071768] (biological process) Relationships: is a type of fatty acid biosynthetic process [GO:0006633]; is a type of cell wall macromolecule biosynthetic process [GO:0044038]; is part of Actinobacterium-type cell wall biogenesis [GO:0071766] Also known as: mycolate biosynthetic process, mycolic acid anabolism, mycolic acid biosynthesis, mycolic acid formation, mycolic acid synthesis References: PMID:15653820 Sources: GOC:mah, MetaCyc:PWYG-321 Definition: The chemical reactions and pathways resulting in the formation of mycolic acids, beta-hydroxy fatty acids with a long alpha-alkyl side chain.